{
  "gene": "UniProtKB:Q13557",
  "gene_name": "Calcium_calmodulin-dependent protein kinase type II subunit delta",
  "term_id": "GO:0004683",
  "term_label": "calcium/calmodulin-dependent protein kinase activity",
  "gene_symbol": "CAMK2D"
}